{
  "gene_name": "POTE ankyrin domain family member G",
  "term_label": "Unknown molecular function",
  "gene_symbol": "POTEG",
  "term_id": "UNKNOWN:0001",
  "gene": "UniProtKB:Q6S5H5"
}